{
  "gene": "UniProtKB:Q63HK5",
  "term_label": "regulation of respiratory gaseous exchange by nervous system process",
  "gene_name": "Teashirt homolog 3",
  "gene_symbol": "TSHZ3",
  "term_id": "GO:0002087"
}